{
  "gene_symbol": "KIF1A",
  "gene": "UniProtKB:Q12756",
  "term_id": "GO:0016192",
  "gene_name": "Kinesin-like protein KIF1A",
  "term_label": "vesicle-mediated transport"
}